altruistic, chimeric sorocarp development [GO:0099138] (biological process) References: PMID:18272966 Definition: Development of a chimeric sorocarp in which cells of all genotypes have an equal chance of becoming a spore cell. Relationships: is a type of GO:0099134; is a type of GO:0099137 Also known as: fully co-operative, chimeric sorocarp development